{
  "gene_name": "Hemopexin",
  "term_id": "UNKNOWN:0001",
  "gene": "UniProtKB:P02790",
  "term_label": "Unknown molecular function",
  "gene_symbol": "HPX"
}